{
  "term_label": "plasma membrane",
  "gene_name": "Disintegrin and metalloproteinase domain-containing protein 18",
  "term_id": "GO:0005886",
  "gene_symbol": "ADAM18",
  "gene": "UniProtKB:Q9Y3Q7"
}